peristalsis [GO:0030432] (biological process) Subtypes: GO:0072105 Relationships: is a type of phasic smooth muscle contraction [GO:0014821] Sources: ISBN:0198506732 Definition: A wavelike sequence of involuntary muscular contraction and relaxation that passes along a tubelike structure, such as the intestine, impelling the contents onwards.